bundle of His cell-Purkinje myocyte adhesion involved in cell communication [GO:0086073] (biological process) Relationships: is a type of GO:0034113; is a type of cardiac muscle cell-cardiac muscle cell adhesion [GO:0086042]; is part of bundle of His cell to Purkinje myocyte communication [GO:0086069] Sources: GOC:BHF, GOC:mtg_cardiac_conduct_nov11 Definition: The attachment of a bundle of His cell to a Purkinje myocyte via adhesion molecules that results in the cells being juxtaposed so that they can communicate.